regulation of MyD88-dependent toll-like receptor signaling pathway [GO:0034124] (biological process) References: PMID:16551253, PMID:17328678 Sources: GOC:add Subtypes: negative regulation of MyD88-dependent toll-like receptor signaling pathway [GO:0034125], positive regulation of MyD88-dependent toll-like receptor signaling pathway [GO:0034126] Also known as: regulation ofMyD88-dependent TLR signaling pathway, regulation ofMyD88-dependent toll-like receptor signalling pathway Definition: Any process that modulates the frequency, rate, or extent of MyD88-dependent toll-like receptor signaling pathway. Relationships: is a type of GO:0034121; regulates MyD88-dependent toll-like receptor signaling pathway [GO:0002755]